{
  "term_label": "positive regulation of DNA-templated transcription",
  "gene_name": "WW domain-binding protein 2",
  "gene": "UniProtKB:Q969T9",
  "gene_symbol": "WBP2",
  "term_id": "GO:0045893"
}